{
  "term_label": "plasma membrane",
  "gene_name": "Catenin delta-2",
  "term_id": "GO:0005886",
  "gene": "UniProtKB:Q9UQB3",
  "gene_symbol": "CTNND2"
}